protein activation cascade [GO:0072376] (biological process) Regulation: regulated by regulation of protein activation cascade [GO:2000257]; negatively regulated by negative regulation of protein activation cascade [GO:2000258]; positively regulated by positive regulation of protein activation cascade [GO:2000259] Subtypes: kinin cascade [GO:0002254], GO:0007597, blood coagulation, extrinsic pathway [GO:0007598], GO:0072377, blood coagulation, fibrin clot formation [GO:0072378], Toll receptor ligand protein activation cascade [GO:0160032] Also known as: protein activation pathway, protein activitory cascade Relationships: is a type of protein maturation [GO:0051604] Sources: GOC:add, GOC:mah, GOC:pde Definition: A sequential series of modifications to a set of proteins where the product of one reaction catalyzes the following reaction, ultimately leading to the generation of a mature protein. Modifications typically include proteolysis or covalent modification, and may also include binding events.